{
  "term_label": "cell surface receptor signaling pathway",
  "gene_symbol": "TRBV10-3",
  "term_id": "GO:0007166",
  "gene": "UniProtKB:A0A0K0K1G6",
  "gene_name": "T cell receptor beta variable 10-3"
}